myosin II tail binding [GO:0032035] (MF) Relationships: is a type of myosin tail binding [GO:0032029]; is a type of GO:0032038 Sources: GOC:mah Definition: Binding to the tail region of a myosin II heavy chain.